regulation of phosphate transmembrane transport [GO:2000185] (BP) Subtypes: negative regulation of phosphate transmembrane transport [GO:2000186], positive regulation of phosphate transmembrane transport [GO:2000187] Relationships: is a type of regulation of phosphate transport [GO:0010966]; is a type of regulation of transmembrane transport [GO:0034762]; regulates phosphate ion transmembrane transport [GO:0035435] Also known as: regulation of phosphate membrane transport Sources: GOC:obol Definition: Any process that modulates the frequency, rate or extent of phosphate transmembrane transport.